Mad-Max complex [GO:0070443] (cellular component) Definition: A transcriptional repressor complex that consists of a heterodimer of the bHLH-ZIP proteins Mad and Max. Relationships: is a type of RNA polymerase II transcription repressor complex [GO:0090571] References: PMID:8224841